{
  "gene_name": "Voltage-dependent calcium channel gamma-6 subunit",
  "term_id": "GO:0005246",
  "gene_symbol": "CACNG6",
  "term_label": "calcium channel regulator activity",
  "gene": "UniProtKB:Q9BXT2"
}